{
  "term_id": "UNKNOWN:0002",
  "gene_symbol": "SLC29A4",
  "gene_name": "Equilibrative nucleoside transporter 4",
  "term_label": "Unknown biological process",
  "gene": "UniProtKB:Q7RTT9"
}